{
  "gene_name": "Keratin, type I cuticular Ha5",
  "gene_symbol": "KRT35",
  "term_label": "keratin filament",
  "term_id": "GO:0045095",
  "gene": "UniProtKB:Q92764"
}